{
  "term_label": "voltage-gated sodium channel complex",
  "gene_name": "Sodium channel protein type 4 subunit alpha",
  "gene_symbol": "SCN4A",
  "gene": "UniProtKB:P35499",
  "term_id": "GO:0001518"
}